chlorate reductase activity [GO:0047143] (molecular function) Also known as: chlorate reductase C, chlorite:acceptor oxidoreductase activity Sources: EC:1.97.1.1, RHEA:16349 Relationships: is a type of oxidoreductase activity [GO:0016491] Definition: Catalysis of the reaction: AH(2) + chlorate = A + chlorite + H2O + H+.